skeletal muscle cell proliferation [GO:0014856] (biological process) Relationships: is a type of GO:0014855 Sources: CL:0000188, GOC:ef, GOC:mtg_muscle Regulation: regulated by regulation of skeletal muscle cell proliferation [GO:0014857]; positively regulated by positive regulation of skeletal muscle cell proliferation [GO:0014858]; negatively regulated by negative regulation of skeletal muscle cell proliferation [GO:0014859] Definition: The multiplication or reproduction of skeletal muscle cells, resulting in the expansion of a cell population. Subtypes: skeletal muscle satellite cell proliferation [GO:0014841]